{
  "gene_symbol": "LRRC59",
  "term_label": "cytoplasm",
  "gene": "UniProtKB:Q96AG4",
  "gene_name": "Leucine-rich repeat-containing protein 59",
  "term_id": "GO:0005737"
}